interleukin-10 receptor activity [GO:0004920] (molecular function) Relationships: is a type of GO:0004896; BFO_0000051 GO:0019969 Sources: GOC:jl, GOC:signaling Definition: Combining with interleukin-10 and transmitting the signal from one side of the membrane to the other to initiate a change in cell activity. Also known as: IL-10 receptor activity, IL-10R